{
  "term_label": "extracellular space",
  "gene": "UniProtKB:Q9H2X0",
  "term_id": "GO:0005615",
  "gene_name": "Chordin",
  "gene_symbol": "CHRD"
}